{
  "term_label": "detection of chemical stimulus involved in sensory perception of smell",
  "term_id": "GO:0050911",
  "gene_symbol": "OR2T5",
  "gene_name": "Olfactory receptor 2T5",
  "gene": "UniProtKB:Q6IEZ7"
}